{
  "term_label": "negative regulation of BMP signaling pathway",
  "gene_name": "Ski oncogene",
  "gene": "UniProtKB:P12755",
  "gene_symbol": "SKI",
  "term_id": "GO:0030514"
}